positive regulation of positive chemotaxis to cAMP by chlorinated alkylphenone [GO:0061124] (biological process) Sources: GOC:dph Definition: Any process that increases the rate, frequency, or extent of directed movement of a motile cell or organism up a concentration gradient of 3',5'-cAMP by the action of a chlorinated alkylphenone. An alkylphenone is an aromatic polyketide with methyl and chlorine substitutions. Relationships: is a type of GO:0061119; is a type of positive regulation of positive chemotaxis to cAMP [GO:0061122] Subtypes: positive regulation of positive chemotaxis to cAMP by DIF-1 [GO:0061126], positive regulation of chemotaxis to cAMP by DIF-2 [GO:0061128]